{
  "term_label": "histone binding",
  "term_id": "GO:0042393",
  "gene_name": "Sterile alpha motif domain-containing protein 11",
  "gene": "UniProtKB:Q96NU1",
  "gene_symbol": "SAMD11"
}